{
  "term_label": "Unknown biological process",
  "gene": "UniProtKB:Q8IUH2",
  "gene_symbol": "CREG2",
  "gene_name": "Protein CREG2",
  "term_id": "UNKNOWN:0002"
}